{
  "term_id": "UNKNOWN:0002",
  "gene_name": "Putative FK506-binding protein 9-like protein",
  "gene": "UniProtKB:Q75LS8",
  "term_label": "Unknown biological process",
  "gene_symbol": "FKBP9P1"
}